{
  "term_label": "Unknown biological process",
  "gene_symbol": "MUCL3",
  "gene": "UniProtKB:Q3MIW9",
  "term_id": "UNKNOWN:0002",
  "gene_name": "Mucin-like protein 3"
}